chloroplast intermembrane space [GO:0031972] (cellular component) Also known as: chloroplast envelope lumen Sources: GOC:mah Definition: The region between the inner and outer lipid bilayers of a chloroplast envelope. Relationships: is a type of plastid intermembrane space [GO:0009529]; is part of chloroplast envelope [GO:0009941]